{
  "gene_symbol": "ATP5ME",
  "gene_name": "ATP synthase subunit e, mitochondrial",
  "gene": "UniProtKB:P56385",
  "term_id": "GO:0042776",
  "term_label": "proton motive force-driven mitochondrial ATP synthesis"
}